{
  "gene_symbol": "SEC31B",
  "gene": "UniProtKB:Q9NQW1",
  "term_id": "GO:0007029",
  "gene_name": "Protein transport protein Sec31B",
  "term_label": "endoplasmic reticulum organization"
}